{
  "term_id": "GO:0005739",
  "term_label": "mitochondrion",
  "gene": "UniProtKB:Q9BT17",
  "gene_name": "Mitochondrial ribosome-associated GTPase 1",
  "gene_symbol": "MTG1"
}